{
  "term_label": "Unknown biological process",
  "gene_name": "Caveolae-associated protein 2",
  "gene": "UniProtKB:O95810",
  "gene_symbol": "CAVIN2",
  "term_id": "UNKNOWN:0002"
}